5-amino-1-ribofuranosylimidazole-4-carboxamide transmembrane transporter activity [GO:1903089] (molecular function) Definition: Enables the transfer of 5-amino-1-ribofuranosylimidazole-4-carboxamide from one side of a membrane to the other. Relationships: is_a GO:0042887; is a type of azole transmembrane transporter activity [GO:1901474]; is a type of carbohydrate derivative transmembrane transporter activity [GO:1901505]; is part of 5-amino-1-ribofuranosylimidazole-4-carboxamide transmembrane transport [GO:1903088] References: PMID:24778186 Sources: GOC:TermGenie, GO_REF:0000066 Also known as: acadesine transporter activity